mitochondrial lysyl-tRNA aminoacylation [GO:0070154] (biological process) Sources: GOC:mah, GOC:mcc Definition: The process of coupling lysine to lysyl-tRNA in a mitochondrion, catalyzed by lysyl-tRNA synthetase. In tRNA aminoacylation, the amino acid is first activated by linkage to AMP and then transferred to either the 2'- or the 3'-hydroxyl group of the 3'-adenosine residue of the tRNA. Relationships: is a type of GO:0006430; is_a tRNA aminoacylation for mitochondrial protein translation [GO:0070127]